pellicular membrane [GO:0120267] (cellular component) Relationships: is a type of plasma membrane region [GO:0098590]; is part of pellicle [GO:0020039] Definition: The portion of the plasma membrane surrounding the pellicle, a structure enclosing some parasite cells such as certain apicomplexa and Euglenozoa. These membranes are associated with an infrastructure of microtubules, microfilaments, and other organelles. Also known as: pellicle membrane, pellicular plasma membrane References: PMID:18095354, PMID:30550896, PMID:6993644, PMID:7175771 Sources: GOC:ach, GOC:krc Note: This sub-domain of the plasma membrane excludes the ciliary and ciliary pocket membranes.